{
  "term_id": "UNKNOWN:0002",
  "term_label": "Unknown biological process",
  "gene_symbol": "PPP1R8",
  "gene": "UniProtKB:Q12972",
  "gene_name": "Nuclear inhibitor of protein phosphatase 1"
}